{
  "term_id": "GO:0045095",
  "gene_symbol": "FAM83H",
  "gene_name": "Protein FAM83H",
  "gene": "UniProtKB:Q6ZRV2",
  "term_label": "keratin filament"
}